leukotriene B4 12-hydroxy dehydrogenase activity [GO:0097257] (molecular function) Definition: Catalysis of the reaction: leukotriene B4 + NADP+ = 12-oxo-leukotriene B4 + NADPH + H+. References: PMID:8394361, PMID:9461497 Sources: GOC:mw, KEGG_REACTION:R03864 Also known as: leukotriene B4 12-hydroxydehydrogenase activity Relationships: is a type of oxidoreductase activity, acting on CH-OH group of donors [GO:0016614]